{
  "gene_name": "Protein MGARP",
  "term_id": "UNKNOWN:0002",
  "term_label": "Unknown biological process",
  "gene_symbol": "MGARP",
  "gene": "UniProtKB:Q8TDB4"
}